{
  "term_id": "GO:0038110",
  "gene_name": "Interleukin-2",
  "term_label": "interleukin-2-mediated signaling pathway",
  "gene_symbol": "IL2",
  "gene": "UniProtKB:P60568"
}